3-deoxyoctulosonase activity [GO:0050534] (molecular function) Definition: Catalysis of the reaction: 3-deoxyoctulosonyl-lipopolysaccharide + H2O = 3-deoxyoctulosonic acid + lipopolysaccharide. Also known as: 3-deoxyoctulosonyl-lipopolysaccharide hydrolase activity, alpha-Kdo-ase activity Relationships: is a type of GO:0004553 Sources: EC:3.2.1.144